{
  "term_id": "GO:0047179",
  "gene_symbol": "PAFAH1B3",
  "gene": "UniProtKB:Q15102",
  "term_label": "platelet-activating factor acetyltransferase activity",
  "gene_name": "Platelet-activating factor acetylhydrolase IB subunit alpha1"
}